{
  "gene_name": "ADP-ribosylation factor-like protein 9",
  "gene": "UniProtKB:Q6T311",
  "term_label": "Unknown cellular component",
  "term_id": "UNKNOWN:0003",
  "gene_symbol": "ARL9"
}